cellular response to wortmannin [GO:1904568] (biological process) Definition: Any process that results in a change in state or activity of a cell (in terms of movement, secretion, enzyme production, gene expression, etc.) as a result of a wortmannin stimulus. References: PMID:20629186 Sources: GOC:TermGenie, GO_REF:0000071 Relationships: is_a GO:1901655; is a type of GO:1904567 Also known as: cellular response to wartmannin